{
  "gene_symbol": "USP17L17",
  "gene": "UniProtKB:D6RBQ6",
  "term_label": "cysteine-type deubiquitinase activity",
  "gene_name": "Ubiquitin carboxyl-terminal hydrolase 17-like protein 17",
  "term_id": "GO:0004843"
}